{
  "gene": "UniProtKB:P33240",
  "gene_name": "Cleavage stimulation factor subunit 2",
  "term_label": "Unknown biological process",
  "gene_symbol": "CSTF2",
  "term_id": "UNKNOWN:0002"
}